{
  "term_id": "UNKNOWN:0001",
  "gene_name": "Protein broad-minded",
  "term_label": "Unknown molecular function",
  "gene_symbol": "TBC1D32",
  "gene": "UniProtKB:Q96NH3"
}